deoxyribonucleoside binding [GO:0032546] (molecular function) Subtypes: purine deoxyribonucleoside binding [GO:0032547], pyrimidine deoxyribonucleoside binding [GO:0032548] Sources: GOC:mah Definition: Binding to a deoxyribonucleoside, a compound consisting of a purine or pyrimidine nitrogenous base linked to deoxyribose. Relationships: is a type of nucleoside binding [GO:0001882]